{
  "gene_symbol": "DNALI1",
  "gene_name": "Axonemal dynein light intermediate polypeptide 1",
  "term_label": "axoneme",
  "gene": "UniProtKB:O14645",
  "term_id": "GO:0005930"
}